regulation of mating-type specific transcription, DNA-templated [GO:0007532] (biological process) Also known as: mating-type specific transcriptional control, regulation of mating-type specific transcription, DNA-dependent Subtypes: negative regulation of mating-type specific transcription, DNA-templated [GO:0045894], positive regulation of mating-type specific transcription, DNA-templated [GO:0045895] Sources: GOC:go_curators, GOC:txnOH Definition: Any mating-type specific process that modulates the frequency, rate or extent of cellular DNA-templated transcription. Relationships: is a type of regulation of DNA-templated transcription [GO:0006355]; is a type of mating type determination [GO:0007531]